{
  "gene_symbol": "SLC51B",
  "term_label": "bile acid secretion",
  "term_id": "GO:0032782",
  "gene_name": "Organic solute transporter subunit beta",
  "gene": "UniProtKB:Q86UW2"
}